eRF1 methyltransferase complex [GO:0035657] (cellular component) References: PMID:17008308, PMID:20400505 Sources: GOC:rb Also known as: eRF1 MTase complex Definition: A protein complex required for the methylation of a glutamine (Gln) residue in the protein release factor eRF1. In S. cerevisiae, this complex consists of at least Trm112p and Mtq2p. Relationships: is a type of methyltransferase complex [GO:0034708]